{
  "gene": "UniProtKB:Q12873",
  "term_label": "histone binding",
  "gene_symbol": "CHD3",
  "gene_name": "Chromodomain-helicase-DNA-binding protein 3",
  "term_id": "GO:0042393"
}